{
  "term_id": "GO:0006357",
  "term_label": "regulation of transcription by RNA polymerase II",
  "gene_symbol": "ZFP30",
  "gene": "UniProtKB:Q9Y2G7",
  "gene_name": "Zinc finger protein 30 homolog"
}